{
  "gene_name": "Kelch-like protein 41",
  "gene_symbol": "KLHL41",
  "term_id": "GO:0033017",
  "gene": "UniProtKB:O60662",
  "term_label": "sarcoplasmic reticulum membrane"
}